{
  "term_label": "Unknown cellular component",
  "gene_symbol": "OR5B3",
  "gene_name": "Olfactory receptor 5B3",
  "gene": "UniProtKB:Q8NH48",
  "term_id": "UNKNOWN:0003"
}